negative regulation of antisense RNA transcription [GO:0060195] (biological process) References: PMID:18075583 Sources: GOC:dph, GOC:tb Relationships: is_a negative regulation of DNA-templated transcription [GO:0045892]; is a type of regulation of antisense RNA transcription [GO:0060194]; negatively regulates antisense RNA transcription [GO:0009300] Definition: Any process that decreases the frequency, rate or extent of the synthesis of antisense RNA, an RNA molecule complementary in sequence to another RNA or DNA molecule, which, by binding the latter, acts to inhibit its function and/or completion of synthesis, on a template of DNA.